{
  "gene_name": "Alpha-ketoglutarate-dependent dioxygenase FTO",
  "term_id": "GO:0005634",
  "gene_symbol": "FTO",
  "gene": "UniProtKB:Q9C0B1",
  "term_label": "nucleus"
}